death effector domain binding [GO:0035877] (molecular function) Note: For binding to the death domain, consider instead the term 'death domain binding ; GO:0070513'. Definition: Binding to a DED domain (death effector domain) of a protein, a homotypic protein interaction module composed of a bundle of six alpha-helices that is related in structure to the death domain (DD). Relationships: is a type of protein domain specific binding [GO:0019904] Also known as: DED binding Sources: GOC:ecd, InterPro:IPR001875